{
  "gene_symbol": "XYLT1",
  "term_label": "heparan sulfate proteoglycan biosynthetic process",
  "term_id": "GO:0015012",
  "gene": "UniProtKB:Q86Y38",
  "gene_name": "Xylosyltransferase 1"
}